{
  "term_id": "UNKNOWN:0003",
  "term_label": "Unknown cellular component",
  "gene_name": "Tetratricopeptide repeat protein 27",
  "gene_symbol": "TTC27",
  "gene": "UniProtKB:Q6P3X3"
}